D-alanine transmembrane transporter activity [GO:0042944] (molecular function) Also known as: D-alanine transporter activity Definition: Enables the transfer of D-alanine from one side of a membrane to the other. D-alanine is the D-enantiomer of 2-aminopropanoic acid. Relationships: is a type of GO:0022858; is a type of GO:0042943; BFO_0000050 D-alanine transmembrane transport [GO:0042941] Sources: GOC:jl, GOC:mtg_transport, ISBN:0815340729